{
  "term_label": "plasma membrane",
  "gene_symbol": "CHRNB3",
  "gene_name": "Neuronal acetylcholine receptor subunit beta-3",
  "term_id": "GO:0005886",
  "gene": "UniProtKB:Q05901"
}